{
  "gene": "UniProtKB:Q08188",
  "term_id": "GO:0018149",
  "gene_name": "Protein-glutamine gamma-glutamyltransferase E",
  "gene_symbol": "TGM3",
  "term_label": "peptide cross-linking"
}